chemoattraction involved in interneuron migration from the subpallium to the cortex [GO:0021841] (biological process) Relationships: is a type of GO:0050918; is part of directional guidance of interneurons involved in migration from the subpallium to the cortex [GO:0021840] Definition: The creation and reception of signals that result in the movement of interneurons toward the signal, where this process is involved in migration from the subpallium to the cortex. Also known as: positive chemotaxis involved in interneuron migration from the subpallium to the cortex References: PMID:12626695 Sources: GOC:cls, GOC:dgh, GOC:dph, GOC:jid, GO_REF:0000021